{
  "gene_symbol": "SEC14L4",
  "gene": "UniProtKB:Q9UDX3",
  "term_label": "Unknown molecular function",
  "gene_name": "SEC14-like protein 4",
  "term_id": "UNKNOWN:0001"
}